anthocyanin accumulation in tissues in response to UV light [GO:0043481] (biological process) Definition: The aggregation of the pigment anthocyanin in a particular location in a tissue, occurring in response to a UV light stimulus. Sources: GOC:jl Relationships: is a type of pigment accumulation in tissues in response to UV light [GO:0043479]